{
  "term_id": "GO:0005886",
  "term_label": "plasma membrane",
  "gene_symbol": "PIEZO2",
  "gene_name": "Piezo-type mechanosensitive ion channel component 2",
  "gene": "UniProtKB:Q9H5I5"
}